regulation of maltopentaose transport [GO:1900315] (biological process) Relationships: is a type of regulation of pentasaccharide transport [GO:1900360]; regulates maltopentaose transport [GO:2001101] Sources: GOC:TermGenie, GOC:mengo_curators Subtypes: negative regulation of maltopentaose transport [GO:1900316], GO:1900317 Definition: Any process that modulates the frequency, rate or extent of maltopentaose transport.